intracellular membraneless organelle [GO:0043232] (cellular component) Definition: Organized structure of distinctive morphology and function, not bounded by a lipid bilayer membrane and occurring within the cell. Includes ribosomes, the cytoskeleton and chromosomes. Also known as: intracellular non-membrane-bounded organelle, intracellular non-membrane-enclosed organelle Subtypes: kinetochore [GO:0000776], podosome [GO:0002102], chromosome [GO:0005694], nucleolus [GO:0005730], lipid droplet [GO:0005811], centriole [GO:0005814], aster [GO:0005818], spindle [GO:0005819], ribosome [GO:0005840], cytoskeleton [GO:0005856], thylakoid [GO:0009579], GO:0010369, nuclear body [GO:0016604], gas vesicle [GO:0031411], bacterial microcompartment [GO:0031469], GO:0032019, GO:0034515, GO:0035770, nematocyst [GO:0042151], mitochondrial nucleoid [GO:0042645], plastid nucleoid [GO:0042646], contractile muscle fiber [GO:0043292], GO:0043590, crystalloid [GO:0044312], GO:0045170, chlorosome [GO:0046858], contractile vacuole complex [GO:0062159], ventral disc [GO:0097597], blepharoplast [GO:0097727], deuterosome [GO:0098536], goblet cell theca [GO:0098593], synaptic ribbon [GO:0098681], arciform density [GO:0098682], GO:0099091, dynein axonemal particle [GO:0120293], cytoplasmic lattice [GO:0140095], protein aggregate center [GO:0140453], GO:0140737, GO:1990732, nucleolus-like body [GO:1990934], transmembrane actin-associated (TAN) line [GO:1990973] Sources: GOC:go_curators Relationships: is a type of GO:0043228; is a type of intracellular organelle [GO:0043229]